plastid localization [GO:0051644] (BP) Sources: GOC:ai Definition: Any process in which a plastid is transported to, and/or maintained in, a specific location within the cell. Also known as: establishment and maintenance of plastid localization, plastid localisation Subtypes: chloroplast localization [GO:0019750], establishment of plastid localization [GO:0051667], maintenance of plastid location [GO:0051688] Relationships: is a type of organelle localization [GO:0051640]